{
  "gene": "UniProtKB:Q8TAV5",
  "term_id": "UNKNOWN:0001",
  "gene_name": "Uncharacterized protein KCNJ5-AS1",
  "term_label": "Unknown molecular function",
  "gene_symbol": "KCNJ5-AS1"
}